response to disaccharide [GO:0034285] (biological process) Definition: Any process that results in a change in state or activity of a cell or an organism (in terms of movement, secretion, enzyme production, gene expression, etc.) as a result of a disaccharide stimulus. Sources: GOC:sart Relationships: is a type of response to carbohydrate [GO:0009743] Subtypes: response to sucrose [GO:0009744], GO:0010353, GO:0034286, detection of disaccharide stimulus [GO:0034288], GO:0071324 Also known as: response to disaccharide stimulus